{
  "term_id": "UNKNOWN:0001",
  "term_label": "Unknown molecular function",
  "gene_name": "Uncharacterized protein encoded by LINC02872",
  "gene": "UniProtKB:A2RU37",
  "gene_symbol": "LINC02872"
}